{
  "term_label": "Unknown biological process",
  "gene": "UniProtKB:Q96LL9",
  "gene_symbol": "DNAJC30",
  "term_id": "UNKNOWN:0002",
  "gene_name": "DnaJ homolog subfamily C member 30, mitochondrial"
}